{
  "term_id": "GO:0005634",
  "gene": "UniProtKB:Q8TD26",
  "gene_name": "Chromodomain-helicase-DNA-binding protein 6",
  "term_label": "nucleus",
  "gene_symbol": "CHD6"
}